{
  "gene_name": "Zinc finger protein 618",
  "gene": "UniProtKB:Q5T7W0",
  "gene_symbol": "ZNF618",
  "term_id": "UNKNOWN:0002",
  "term_label": "Unknown biological process"
}